regulation of antimicrobial humoral response [GO:0002759] (biological process) Subtypes: GO:0002760, GO:0002784, GO:0008348 Definition: Any process that modulates the frequency, rate, or extent of an antimicrobial humoral response. Sources: GOC:add Relationships: is a type of regulation of response to biotic stimulus [GO:0002831]; is a type of regulation of humoral immune response [GO:0002920]; is a type of regulation of defense response [GO:0031347]; is a type of regulation of response to external stimulus [GO:0032101]; regulates antimicrobial humoral response [GO:0019730]